{
  "term_id": "GO:0000978",
  "gene_symbol": "IRF6",
  "term_label": "RNA polymerase II cis-regulatory region sequence-specific DNA binding",
  "gene": "UniProtKB:O14896",
  "gene_name": "Interferon regulatory factor 6"
}